{
  "term_id": "GO:0045087",
  "gene_name": "Tripartite motif-containing protein 6",
  "gene_symbol": "TRIM6",
  "gene": "UniProtKB:Q9C030",
  "term_label": "innate immune response"
}